{
  "gene_symbol": "AXL",
  "gene": "UniProtKB:P30530",
  "term_label": "phagocytosis",
  "gene_name": "Tyrosine-protein kinase receptor UFO",
  "term_id": "GO:0006909"
}